{
  "gene_name": "Methenyltetrahydrofolate synthase domain-containing protein",
  "gene": "UniProtKB:Q2M296",
  "gene_symbol": "MTHFSD",
  "term_id": "UNKNOWN:0001",
  "term_label": "Unknown molecular function"
}